bacterial-type flagellum secretion apparatus [GO:0120102] (cellular component) References: PMID:10572114, PMID:12624192, PMID:24697492, PMID:25251856 Sources: DOI:10.1002/9780470015902.a0000744.pub4, GOC:cilia Definition: A part of the bacterial-type flagellum that is located at the cytoplasmic side of the MS ring and composed of six membrane proteins (FlhA, FlhB, FliP, FliQ, FliR, and FliO, or orthologs thereof) and three soluble proteins (FliI, FliH, and FliJ, or orthologs thereof) in the cytoplasm. It is responsible for secretion of flagellar type III protein substrates, including the proteins of the flagellar rod, hook, and filament. Relationships: is a type of cellular anatomical structure [GO:0110165]; is part of bacterial-type flagellum basal body [GO:0009425] Also known as: bacterial-type flagellum export apparatus